{
  "term_label": "Unknown molecular function",
  "term_id": "UNKNOWN:0001",
  "gene_name": "Intraflagellar transport protein 57 homolog",
  "gene_symbol": "IFT57",
  "gene": "UniProtKB:Q9NWB7"
}